{
  "term_label": "RNA binding",
  "gene": "UniProtKB:Q9UNX3",
  "gene_name": "Ribosomal protein uL24-like",
  "gene_symbol": "RPL26L1",
  "term_id": "GO:0003723"
}